{
  "gene_symbol": "TET2",
  "gene_name": "Methylcytosine dioxygenase TET2",
  "gene": "UniProtKB:Q6N021",
  "term_id": "GO:0045944",
  "term_label": "positive regulation of transcription by RNA polymerase II"
}